{
  "gene": "UniProtKB:Q96R47",
  "term_label": "detection of chemical stimulus involved in sensory perception of smell",
  "gene_symbol": "OR2A14",
  "gene_name": "Olfactory receptor 2A14",
  "term_id": "GO:0050911"
}